{
  "gene_name": "Testis-specific Y-encoded protein 4",
  "term_id": "GO:0042393",
  "gene": "UniProtKB:P0CV99",
  "term_label": "histone binding",
  "gene_symbol": "TSPY4"
}